{
  "gene_symbol": "TRBV6-1",
  "gene_name": "T cell receptor beta variable 6-1",
  "gene": "UniProtKB:A0A0K0K1D8",
  "term_label": "Unknown molecular function",
  "term_id": "UNKNOWN:0001"
}